{
  "gene_symbol": "LOXL1",
  "term_label": "extracellular matrix",
  "gene_name": "Lysyl oxidase homolog 1",
  "term_id": "GO:0031012",
  "gene": "UniProtKB:Q08397"
}